{
  "gene_name": "Cyclin-G-associated kinase",
  "term_label": "clathrin binding",
  "gene": "UniProtKB:O14976",
  "gene_symbol": "GAK",
  "term_id": "GO:0030276"
}